symbiont-mediated suppression of host CRISPR-cas system [GO:0098672] (BP) Definition: A process by which a symbiont inhibits or disrupts the CRISPR-cas system of its host. Bacteria and archaea use CRISPR-Cas adaptive immune systems to defend themselves from infection by bacteriophages (phages), and phages have various mechanisms to counter the CRISPR-cas system. References: PMID:23242138, PMID:23446421, PMID:26416740, PMID:28749735 Also known as: anti-CRISPR, CRISPR-cas system evasion by virus, suppression of host CRISPR-cas system, evasion by virus of CRISPR-cas system, inhibition of host CRISPR-cas system by virus Relationships: is_a GO:0052031